peptidyl-lysine N6-acetylation [GO:0018003] (biological process) Relationships: is a type of internal peptidyl-lysine acetylation [GO:0018393] Note: See also the molecular function term 'tubulin N-acetyltransferase activity ; GO:0019799'. Definition: The acetylation of the peptidyl-lysine of proteins to form the derivative peptidyl-N6-acetyl-L-lysine. Sources: RESID:AA0055